{
  "gene": "UniProtKB:Q8WYL5",
  "term_id": "GO:0003779",
  "gene_name": "Protein phosphatase Slingshot homolog 1",
  "term_label": "actin binding",
  "gene_symbol": "SSH1"
}